histone H4K20me3 reader activity [GO:1990889] (MF) Also known as: H4K20me3 modified histone binding Definition: A histone reader that recognizes a histone H4 trimethylated at lysine 20. Relationships: is a type of GO:0140008 References: PMID:20943666, PMID:22150589 Note: Note that the residue position corresponds to the canonical human H4 histone (UniProtKB:P02309); this residue is conserved across all eukaryotes. Note that the initiation methionine is cleaved, so the first residue is S1.